{
  "gene_symbol": "CRACD",
  "term_id": "UNKNOWN:0003",
  "gene_name": "Capping protein-inhibiting regulator of actin dynamics",
  "gene": "UniProtKB:Q6ZU35",
  "term_label": "Unknown cellular component"
}